{
  "term_id": "GO:0031424",
  "gene": "UniProtKB:P35908",
  "gene_name": "Keratin, type II cytoskeletal 2 epidermal",
  "gene_symbol": "KRT2",
  "term_label": "keratinization"
}